{
  "gene": "UniProtKB:Q8TC90",
  "gene_name": "Coiled-coil domain-containing glutamate-rich protein 1",
  "gene_symbol": "CCER1",
  "term_label": "Unknown cellular component",
  "term_id": "UNKNOWN:0003"
}